RENT complex [GO:0030869] (cellular component) References: PMID:12196389 Definition: A protein complex that mediates transcriptional silencing at the rDNA locus (the name derives from regulator of nucleolar silencing and telophase). In Saccharomyces the complex contains Net1p, Sir2p, Cdc14p, and at least one more subunit. Relationships: is a type of GO:0005677; BFO_0000050 nucleolus [GO:0005730]